{
  "gene_symbol": "URM1",
  "term_id": "GO:0005634",
  "term_label": "nucleus",
  "gene_name": "Ubiquitin-related modifier 1",
  "gene": "UniProtKB:Q9BTM9"
}